{
  "gene_name": "WAS protein family homolog 6",
  "term_id": "GO:0034314",
  "term_label": "Arp2/3 complex-mediated actin nucleation",
  "gene_symbol": "WASH6P",
  "gene": "UniProtKB:Q9NQA3"
}